{
  "gene_symbol": "EIF3K",
  "term_label": "Unknown biological process",
  "term_id": "UNKNOWN:0002",
  "gene_name": "Eukaryotic translation initiation factor 3 subunit K",
  "gene": "UniProtKB:Q9UBQ5"
}